{
  "gene": "UniProtKB:Q6UB99",
  "term_id": "UNKNOWN:0002",
  "gene_name": "Ankyrin repeat domain-containing protein 11",
  "gene_symbol": "ANKRD11",
  "term_label": "Unknown biological process"
}